{
  "term_id": "UNKNOWN:0002",
  "gene_symbol": "MROH6",
  "term_label": "Unknown biological process",
  "gene": "UniProtKB:A6NGR9",
  "gene_name": "Maestro heat-like repeat-containing protein family member 6"
}